regulation of cardiac muscle cell contraction [GO:0086004] (biological process) Definition: Any process that modulates the frequency, rate or extent of cardiac muscle cell contraction. Subtypes: regulation of atrial cardiac muscle cell action potential [GO:0098910], regulation of ventricular cardiac muscle cell action potential [GO:0098911], positive regulation of cardiac muscle cell contraction [GO:0106134], GO:0106135 Sources: GOC:BHF, GOC:mtg_cardiac_conduct_nov11 Relationships: is a type of regulation of cardiac muscle contraction [GO:0055117]; is a type of regulation of actin filament-based movement [GO:1903115]; regulates cardiac muscle cell contraction [GO:0086003]